{
  "term_id": "UNKNOWN:0002",
  "gene_name": "Keratin-associated protein 10-10",
  "gene_symbol": "KRTAP10-10",
  "term_label": "Unknown biological process",
  "gene": "UniProtKB:P60014"
}